{
  "gene_symbol": "EZH2",
  "gene": "UniProtKB:Q15910",
  "term_label": "histone H3K27 methyltransferase activity",
  "term_id": "GO:0046976",
  "gene_name": "Histone-lysine N-methyltransferase EZH2"
}